{
  "term_label": "mitochondrion",
  "gene_symbol": "PTCD2",
  "gene": "UniProtKB:Q8WV60",
  "term_id": "GO:0005739",
  "gene_name": "Pentatricopeptide repeat-containing protein 2, mitochondrial"
}